vitamin binding [GO:0019842] (molecular function) Definition: Binding to a vitamin, one of a number of unrelated organic substances that occur in many foods in small amounts and that are necessary in trace amounts for the normal metabolic functioning of the body. Relationships: is a type of small molecule binding [GO:0036094] Subtypes: vitamin D binding [GO:0005499], folic acid binding [GO:0005542], GO:0008431, biotin binding [GO:0009374], retinal binding [GO:0016918], retinol binding [GO:0019841], thiamine binding [GO:0030975], thiamine pyrophosphate binding [GO:0030976], GO:0031177, L-ascorbic acid binding [GO:0031418], cobalamin binding [GO:0031419], vitamin B6 binding [GO:0070279] Sources: GOC:ai